{
  "term_id": "GO:0045505",
  "gene_name": "Dynein axonemal heavy chain 8",
  "gene": "UniProtKB:Q96JB1",
  "term_label": "dynein intermediate chain binding",
  "gene_symbol": "DNAH8"
}